pollen tube [GO:0090406] (cellular component) Relationships: is a type of plasma membrane bounded cell projection [GO:0120025] Note: Carries the male gametes to into or near the ovule. May be branched in gymnosperms. This term replaces the obsolete term PO:0006345. Part of pollen tube cell (PO:0025195). Definition: A tubular cell projection that is part of a pollen tube cell and extends from a pollen grain. Sources: GOC:tb, PO:0025195, PO:0025281